CUGBP1-eIF2 complex [GO:0071075] (cellular component) Definition: A protein complex that contains the eukaryotic translation initiation factor 2 complex (EIF2), CUG binding protein 1, and several endoplasmic reticulum proteins; the complex is involved in the regulation of translation. Relationships: is a type of protein-containing complex [GO:0032991]; is part of cytoplasm [GO:0005737] References: PMID:16931514